deaminated glutathione amidase activity [GO:0110050] (molecular function) Definition: Catalysis of the reaction: N-(4-oxoglutarate)-L-cysteinylglycine + H2O = 2-oxoglutarate + L-cysteinylglycine. References: PMID:28373563 Sources: GOC:ka, RHEA:54532 Note: N-(4-oxoglutarate)-L-cysteinylglycine = deaminated glutathione Relationships: is a type of hydrolase activity, acting on carbon-nitrogen (but not peptide) bonds, in linear amides [GO:0016811]